{
  "term_label": "Unknown biological process",
  "gene_symbol": "AKAP5",
  "term_id": "UNKNOWN:0002",
  "gene_name": "A-kinase anchor protein 5",
  "gene": "UniProtKB:P24588"
}